{
  "term_label": "Unknown molecular function",
  "gene_name": "Sushi domain-containing protein 6",
  "gene": "UniProtKB:Q92537",
  "gene_symbol": "SUSD6",
  "term_id": "UNKNOWN:0001"
}